{
  "term_label": "Unknown cellular component",
  "term_id": "UNKNOWN:0003",
  "gene_symbol": "OR5M9",
  "gene_name": "Olfactory receptor 5M9",
  "gene": "UniProtKB:Q8NGP3"
}